cellular response to actin cytoskeletal stress [GO:0120306] (biological process) Relationships: is a type of cellular response to stress [GO:0033554] References: PMID:32915139 Sources: GOC:krc, GOC:vw Also known as: cellular response to actin cytoskeleton stress, cellular response to latrunculin A, cellular response to latrunculin B, response to latrunculin A, response to latrunculin B Definition: Any process that results in a change in state or activity of a cell (in terms of movement, secretion, enzyme production, gene expression, etc.) as a result of perturbations or damage to the actin cytoskeleton.